cellular response to UV-B [GO:0071493] (biological process) Definition: Any process that results in a change in state or activity of a cell (in terms of movement, secretion, enzyme production, gene expression, etc.) as a result of a UV-B radiation stimulus. UV-B radiation (UV-B light) spans the wavelengths 280 to 315 nm. Also known as: cellular response to UV-B light stimulus, cellular response to UV-B radiation stimulus, cellular response to UVB light stimulus, cellular response to UVB radiation stimulus, cellular response to medium wave ultraviolet light stimulus, cellular response to medium wave ultraviolet radiation stimulus Sources: GOC:mah Relationships: is a type of response to UV-B [GO:0010224]; is a type of cellular response to UV [GO:0034644]